{
  "term_id": "UNKNOWN:0002",
  "gene_name": "Wnt inhibitory factor 1",
  "gene_symbol": "WIF1",
  "term_label": "Unknown biological process",
  "gene": "UniProtKB:Q9Y5W5"
}